{
  "gene": "UniProtKB:O95236",
  "term_id": "GO:0008289",
  "term_label": "lipid binding",
  "gene_name": "Apolipoprotein L3",
  "gene_symbol": "APOL3"
}